{
  "term_label": "DNA binding",
  "gene_symbol": "THRAP3",
  "term_id": "GO:0003677",
  "gene": "UniProtKB:Q9Y2W1",
  "gene_name": "Thyroid hormone receptor-associated protein 3"
}